{
  "term_label": "hippo signaling",
  "gene_symbol": "WWTR1",
  "term_id": "GO:0035329",
  "gene_name": "WW domain-containing transcription regulator protein 1",
  "gene": "UniProtKB:Q9GZV5"
}